{
  "term_label": "regulation of receptor signaling pathway via JAK-STAT",
  "term_id": "GO:0046425",
  "gene_name": "Putative macrophage stimulating 1-like protein",
  "gene": "UniProtKB:Q2TV78",
  "gene_symbol": "MST1L"
}